regulation of dendritic cell chemotaxis [GO:2000508] (biological process) Relationships: is a type of regulation of leukocyte chemotaxis [GO:0002688]; is_a regulation of mononuclear cell migration [GO:0071675]; regulates dendritic cell chemotaxis [GO:0002407] Definition: Any process that modulates the frequency, rate or extent of dendritic cell chemotaxis. Subtypes: negative regulation of dendritic cell chemotaxis [GO:2000509], positive regulation of dendritic cell chemotaxis [GO:2000510], GO:2000527 Sources: GOC:obol